{
  "term_label": "BBSome",
  "gene_symbol": "BBS1",
  "gene_name": "Bardet-Biedl syndrome 1 protein",
  "term_id": "GO:0034464",
  "gene": "UniProtKB:Q8NFJ9"
}